protein localization to axon [GO:0099612] (biological process) Subtypes: GO:0002175, GO:0071205 References: PMID:26157139 Sources: GOC:dos Definition: A process in which a protein is transported to or maintained in a location within an axon. Relationships: is a type of intracellular protein localization [GO:0008104]